{
  "term_label": "Unknown cellular component",
  "gene_symbol": "MFHAS1",
  "gene_name": "Malignant fibrous histiocytoma-amplified sequence 1",
  "term_id": "UNKNOWN:0003",
  "gene": "UniProtKB:Q9Y4C4"
}